{
  "gene_name": "Hairy_enhancer-of-split related with YRPW motif protein 2",
  "term_label": "circulatory system development",
  "gene_symbol": "HEY2",
  "gene": "UniProtKB:Q9UBP5",
  "term_id": "GO:0072359"
}